{
  "term_id": "GO:0043235",
  "gene": "UniProtKB:P35590",
  "gene_symbol": "TIE1",
  "gene_name": "Tyrosine-protein kinase receptor Tie-1",
  "term_label": "receptor complex"
}